AMP biosynthetic process [GO:0006167] (biological process) Subtypes: 'de novo' AMP biosynthetic process [GO:0044208], AMP salvage [GO:0044209] Also known as: AMP anabolism, AMP biosynthesis, AMP formation, AMP synthesis Sources: GOC:go_curators, ISBN:0198506732 Relationships: is_a purine ribonucleotide biosynthetic process [GO:0009152]; is a type of purine ribonucleoside monophosphate biosynthetic process [GO:0009168]; is a type of AMP metabolic process [GO:0046033] Definition: The chemical reactions and pathways resulting in the formation of AMP, adenosine monophosphate.